{
  "gene_name": "Vacuolar fusion protein MON1 homolog A",
  "gene": "UniProtKB:Q86VX9",
  "gene_symbol": "MON1A",
  "term_label": "Mon1-Ccz1 complex",
  "term_id": "GO:0035658"
}